{
  "gene_symbol": "SLC4A7",
  "term_id": "GO:0051453",
  "gene_name": "Sodium bicarbonate cotransporter 3",
  "term_label": "regulation of intracellular pH",
  "gene": "UniProtKB:Q9Y6M7"
}